{
  "gene_symbol": "FAM90A14",
  "term_id": "UNKNOWN:0001",
  "gene": "UniProtKB:P0C7W9",
  "gene_name": "Putative protein FAM90A14",
  "term_label": "Unknown molecular function"
}